{
  "gene_name": "Pro-neuropeptide Y",
  "gene_symbol": "NPY",
  "term_id": "GO:0007218",
  "term_label": "neuropeptide signaling pathway",
  "gene": "UniProtKB:P01303"
}